{
  "term_label": "Unknown biological process",
  "gene_name": "Ankyrin repeat domain-containing protein 34A",
  "gene_symbol": "ANKRD34A",
  "gene": "UniProtKB:Q69YU3",
  "term_id": "UNKNOWN:0002"
}